{
  "term_id": "GO:0005654",
  "gene": "UniProtKB:Q5MJ70",
  "gene_name": "Speedy protein A",
  "term_label": "nucleoplasm",
  "gene_symbol": "SPDYA"
}